{
  "term_label": "protein serine/threonine kinase activity",
  "term_id": "GO:0004674",
  "gene_symbol": "CSNK1D",
  "gene_name": "Casein kinase I isoform delta",
  "gene": "UniProtKB:P48730"
}